{
  "gene_symbol": "SAG",
  "gene": "UniProtKB:P10523",
  "gene_name": "S-arrestin",
  "term_label": "photoreceptor inner segment",
  "term_id": "GO:0001917"
}